{
  "gene": "UniProtKB:Q5VU92",
  "gene_symbol": "DCAF12L1",
  "gene_name": "DDB1- and CUL4-associated factor 12-like protein 1",
  "term_id": "UNKNOWN:0001",
  "term_label": "Unknown molecular function"
}